{
  "gene": "UniProtKB:Q9UHW5",
  "term_id": "UNKNOWN:0002",
  "term_label": "Unknown biological process",
  "gene_name": "GPN-loop GTPase 3",
  "gene_symbol": "GPN3"
}